positive regulation of circadian sleep/wake cycle, wakefulness [GO:0010841] (biological process) Relationships: is a type of regulation of circadian sleep/wake cycle, wakefulness [GO:0010840]; is a type of positive regulation of circadian rhythm [GO:0042753]; is a type of positive regulation of behavior [GO:0048520]; positively regulates GO:0042746 Sources: GOC:BHF, GOC:dph, GOC:tb Definition: Any process that increases the frequency, or extent of the wakeful phase of the circadian sleep/wake cycle. The wakeful phase is the part of the circadian sleep/wake cycle where the organism is not asleep.